{
  "gene_name": "Reticulon-1",
  "term_id": "GO:0071787",
  "gene": "UniProtKB:Q16799",
  "term_label": "endoplasmic reticulum tubular network formation",
  "gene_symbol": "RTN1"
}